{
  "gene_name": "Mineralocorticoid receptor",
  "term_label": "regulation of transcription by RNA polymerase II",
  "term_id": "GO:0006357",
  "gene_symbol": "NR3C2",
  "gene": "UniProtKB:P08235"
}